has_alternative_id [oboInOwl#hasAlternativeId]